{
  "gene": "UniProtKB:P07498",
  "gene_name": "Kappa-casein",
  "term_id": "UNKNOWN:0001",
  "gene_symbol": "CSN3",
  "term_label": "Unknown molecular function"
}